{
  "term_label": "plasma membrane",
  "gene_name": "Olfactory receptor 2T3",
  "term_id": "GO:0005886",
  "gene_symbol": "OR2T3",
  "gene": "UniProtKB:Q8NH03"
}